{
  "term_label": "septin complex",
  "gene_name": "Septin-6",
  "gene": "UniProtKB:Q14141",
  "gene_symbol": "SEPTIN6",
  "term_id": "GO:0031105"
}